{
  "gene_name": "Mesoderm induction early response protein 2",
  "term_id": "GO:0003714",
  "gene": "UniProtKB:Q8N344",
  "gene_symbol": "MIER2",
  "term_label": "transcription corepressor activity"
}